{
  "term_label": "regulation of postsynaptic neurotransmitter receptor internalization",
  "gene_name": "IQ motif and SEC7 domain-containing protein 3",
  "term_id": "GO:0099149",
  "gene": "UniProtKB:Q9UPP2",
  "gene_symbol": "IQSEC3"
}